{
  "gene": "UniProtKB:P01920",
  "gene_name": "HLA class II histocompatibility antigen, DQ beta 1 chain",
  "term_label": "MHC class II protein complex",
  "gene_symbol": "HLA-DQB1",
  "term_id": "GO:0042613"
}